{
  "gene": "UniProtKB:P36269",
  "term_id": "GO:0036374",
  "term_label": "glutathione hydrolase activity",
  "gene_symbol": "GGT5",
  "gene_name": "Glutathione hydrolase 5 proenzyme"
}